{
  "gene_symbol": "TP53BP1",
  "gene_name": "TP53-binding protein 1",
  "gene": "UniProtKB:Q12888",
  "term_id": "GO:0042393",
  "term_label": "histone binding"
}